{
  "term_id": "GO:0045663",
  "term_label": "positive regulation of myoblast differentiation",
  "gene_name": "Myogenic factor 6",
  "gene": "UniProtKB:P23409",
  "gene_symbol": "MYF6"
}